dystroglycan complex [GO:0016011] (cellular component) Relationships: is a type of plasma membrane protein complex [GO:0098797]; is part of GO:0016010 Definition: A protein complex that includes alpha- and beta-dystroglycan, which are alternative products of the same gene; the laminin-binding component of the dystrophin-associated glycoprotein complex, providing a link between the subsarcolemmal cytoskeleton (in muscle cells) and the extracellular matrix. Alpha-dystroglycan is an extracellular protein binding to alpha-laminin and to beta-dystroglycan; beta-dystroglycan is a transmembrane protein which binds alpha-dystroglycan and dystrophin. References: PMID:15117830, PMID:16710609